globoside metabolic process [GO:0001575] (biological process) Subtypes: globoside biosynthetic process [GO:0001576] Definition: The chemical reactions and pathways involving globosides, globotetraosylceramides, ceramides containing a core structure of GalNAc-beta-(1->3)-Gal-alpha-(1->4)-Glc(I). Globosides are the major neutral glycosphingolipid in normal kidneys and erythrocytes. Relationships: is a type of GO:0006687 Also known as: globoside metabolism Sources: ISBN:0198506732